epithelium regeneration [GO:1990399] (biological process) Also known as: regeneration of epithelium Subtypes: sensory epithelium regeneration [GO:0070654] Relationships: is a type of tissue regeneration [GO:0042246]; is a type of epithelium development [GO:0060429] Definition: The regrowth of lost or destroyed epithelium. Regulation: regulated by GO:1905041; negatively regulated by GO:1905042; RO_0002213 by GO:1905043 References: PMID:19845688 Sources: GOC:sl